{
  "term_label": "glutamatergic synapse",
  "term_id": "GO:0098978",
  "gene_name": "SLIT-ROBO Rho GTPase-activating protein 2",
  "gene": "UniProtKB:O75044",
  "gene_symbol": "SRGAP2"
}